{
  "gene_symbol": "CRCP",
  "gene": "UniProtKB:O75575",
  "term_id": "GO:0006384",
  "gene_name": "DNA-directed RNA polymerase III subunit RPC9",
  "term_label": "transcription initiation at RNA polymerase III promoter"
}